{
  "gene_symbol": "MANBA",
  "gene_name": "Beta-mannosidase",
  "term_label": "beta-mannosidase activity",
  "gene": "UniProtKB:O00462",
  "term_id": "GO:0004567"
}